H2 histamine receptor binding [GO:0031808] (molecular function) Sources: GOC:mah, GOC:nln Definition: Binding to a H2 histamine receptor. Also known as: H2 histamine receptor ligand Relationships: is a type of G protein-coupled histamine receptor binding [GO:0031806]